diphosphate-fructose-6-phosphate 1-phosphotransferase activity [GO:0047334] (molecular function) Sources: EC:2.7.1.90, MetaCyc:2.7.1.90-RXN Relationships: is a type of phosphofructokinase activity [GO:0008443] Definition: Catalysis of the reaction: fructose-6-phosphate + diphosphate = phosphate + fructose-1,6-bisphosphate. Also known as: 6-phosphofructokinase (diphosphate) activity, 6-phosphofructokinase (pyrophosphate) activity, diphosphate-dependent 6-phosphofructose-1-kinase activity, diphosphate:D-fructose-6-phosphate 1-phosphotransferase activity, inorganic pyrophosphate-dependent phosphofructokinase activity, inorganic pyrophosphate-phosphofructokinase activity, pyrophosphate--fructose 6-phosphate 1-phosphotransferase activity, pyrophosphate-dependent 6-phosphofructose-1-kinase activity, pyrophosphate-dependent phosphofructo-1-kinase activity, pyrophosphate-fructose 6-phosphate phosphotransferase activity